{
  "term_label": "neuronal cell body",
  "gene": "UniProtKB:P54750",
  "term_id": "GO:0043025",
  "gene_name": "Dual specificity calcium_calmodulin-dependent 3',5'-cyclic nucleotide phosphodiesterase 1A",
  "gene_symbol": "PDE1A"
}